inositol hexakisphosphate 1-kinase activity [GO:0052723] (molecular function) Definition: Catalysis of the reaction: 1D-myo-inositol hexakisphosphate + ATP = 1-diphospho-1D-myo-inositol 2,3,4,5,6-pentakisphosphate + ADP. References: PMID:18981179 Sources: RHEA:37459 Relationships: is a type of inositol hexakisphosphate kinase activity [GO:0000828]